regulation of epidermal growth factor receptor signaling pathway involved in heart process [GO:1905282] (biological process) Relationships: is a type of regulation of epidermal growth factor receptor signaling pathway [GO:0042058]; regulates epidermal growth factor receptor signaling pathway involved in heart process [GO:1905251] References: PMID:23069713 Sources: GOC:BHF, GOC:BHF_miRNA, GOC:TermGenie, GOC:bc, GO_REF:0000058 Also known as: regulation of EGF receptor signaling pathway involved in heart process, regulation of EGF receptor signalling pathway involved in heart process, regulation of EGFR signaling pathway involved in heart process, regulation of ERBB1 signaling pathway involved in heart process, regulation of epidermal growth factor receptor signalling pathway involved in heart process, regulation of receptor tyrosine-protein kinase erbB-1 signaling pathway involved in heart process, regulation of EGF receptor signaling pathway involved in cardiac process, regulation of EGF receptor signalling pathway involved in cardiac process, regulation of EGFR signaling pathway involved in cardiac process, regulation of ERBB1 signaling pathway involved in cardiac process, regulation of epidermal growth factor receptor signaling pathway involved in cardiac process, regulation of epidermal growth factor receptor signalling pathway involved in cardiac process, regulation of receptor tyrosine-protein kinase erbB-1 signaling pathway involved in cardiac process Definition: Any process that modulates the frequency, rate or extent of epidermal growth factor receptor signaling pathway involved in heart process. Subtypes: negative regulation of epidermal growth factor receptor signaling pathway involved in heart process [GO:1905283], positive regulation of epidermal growth factor receptor signaling pathway involved in heart process [GO:1905284]